negative regulation of single stranded viral RNA replication via double stranded DNA intermediate [GO:0045869] (biological process) Definition: Any process that stops, prevents, or reduces the frequency, rate or extent of single stranded viral RNA replication via double stranded DNA intermediate. Sources: GOC:go_curators Also known as: down regulation of retroviral genome replication, down-regulation of retroviral genome replication, downregulation of retroviral genome replication, negative regulation of retroviral genome replication, inhibition of retroviral genome replication, regulation of retroviral genome replication Relationships: is a type of negative regulation of viral genome replication [GO:0045071]; is a type of GO:0045091; is a type of negative regulation of RNA biosynthetic process [GO:1902679]; negatively regulates GO:0039692